{
  "gene": "UniProtKB:P18440",
  "gene_name": "Arylamine N-acetyltransferase 1",
  "term_label": "Unknown cellular component",
  "term_id": "UNKNOWN:0003",
  "gene_symbol": "NAT1"
}